{
  "gene_symbol": "GOLGA2",
  "term_label": "mitotic spindle assembly",
  "gene_name": "Golgin subfamily A member 2",
  "gene": "UniProtKB:Q08379",
  "term_id": "GO:0090307"
}